{
  "term_label": "inflammatory response",
  "gene_name": "Eotaxin",
  "gene": "UniProtKB:P51671",
  "term_id": "GO:0006954",
  "gene_symbol": "CCL11"
}